{
  "gene_name": "Leucine-rich repeat-containing protein 31",
  "term_label": "Unknown cellular component",
  "term_id": "UNKNOWN:0003",
  "gene": "UniProtKB:Q6UY01",
  "gene_symbol": "LRRC31"
}